{
  "gene_name": "Protein FAM163A",
  "gene": "UniProtKB:Q96GL9",
  "gene_symbol": "FAM163A",
  "term_id": "UNKNOWN:0002",
  "term_label": "Unknown biological process"
}